{
  "term_label": "signaling receptor binding",
  "term_id": "GO:0005102",
  "gene_name": "Tyrosine-protein kinase FRK",
  "gene_symbol": "FRK",
  "gene": "UniProtKB:P42685"
}